{
  "gene": "UniProtKB:P00558",
  "term_label": "glycolytic process",
  "gene_name": "Phosphoglycerate kinase 1",
  "gene_symbol": "PGK1",
  "term_id": "GO:0006096"
}